{
  "term_id": "GO:0005179",
  "gene": "UniProtKB:P01242",
  "term_label": "hormone activity",
  "gene_symbol": "GH2",
  "gene_name": "Growth hormone variant"
}